{
  "term_label": "Unknown cellular component",
  "gene_name": "Regulation of nuclear pre-mRNA domain-containing protein 1A",
  "gene_symbol": "RPRD1A",
  "term_id": "UNKNOWN:0003",
  "gene": "UniProtKB:Q96P16"
}